{
  "gene_name": "Repulsive guidance molecule A",
  "gene": "UniProtKB:Q96B86",
  "term_id": "GO:0015026",
  "gene_symbol": "RGMA",
  "term_label": "coreceptor activity"
}